regulation of galactoglucomannan catabolic process [GO:2000912] (biological process) Definition: Any process that modulates the frequency, rate or extent of galactoglucomannan catabolic process. Sources: GOC:mengo_curators Also known as: regulation of galactoglucomannan catabolism Relationships: is a type of regulation of polysaccharide metabolic process [GO:0032881]; is a type of regulation of carbohydrate catabolic process [GO:0043470]; regulates galactoglucomannan catabolic process [GO:2000885] Subtypes: negative regulation of galactoglucomannan catabolic process [GO:2000913], positive regulation of galactoglucomannan catabolic process [GO:2000914]